{
  "gene_symbol": "TRAJ57",
  "gene_name": "T cell receptor alpha joining 57 (Fragment)",
  "term_label": "Unknown molecular function",
  "gene": "UniProtKB:A0A075B704",
  "term_id": "UNKNOWN:0001"
}